{
  "gene_name": "Tumor necrosis factor receptor superfamily member 10D",
  "gene": "UniProtKB:Q9UBN6",
  "term_label": "plasma membrane",
  "term_id": "GO:0005886",
  "gene_symbol": "TNFRSF10D"
}